dUTP pyrophosphatase inhibitor activity [GO:0004858] (molecular function) Sources: GOC:mah Definition: Binds to and stops, prevents or reduces the activity of dUTP pyrophosphatase. Relationships: is a type of enzyme inhibitor activity [GO:0004857]; RO_0002212 GO:0004170